{
  "gene_name": "Proline-rich protein 33",
  "gene_symbol": "PRR33",
  "term_id": "UNKNOWN:0002",
  "term_label": "Unknown biological process",
  "gene": "UniProtKB:A8MZF0"
}